{
  "term_id": "GO:0000124",
  "gene": "UniProtKB:P0C7V6",
  "gene_name": "Putative transcription factor SPT20 homolog-like 2",
  "gene_symbol": "SUPT20HL2",
  "term_label": "SAGA complex"
}